{
  "term_id": "UNKNOWN:0002",
  "gene_symbol": "CINP",
  "term_label": "Unknown biological process",
  "gene": "UniProtKB:Q9BW66",
  "gene_name": "Cyclin-dependent kinase 2-interacting protein"
}